histone decrotonylase activity, NAD-dependent [GO:0160012] (molecular function) References: PMID:28497810 Subtypes: histone H3K18 decrotonylase activity [GO:0170012] Definition: Catalysis of the reaction: H2O + N6-(2E)-butenoyl-L-lysyl-[histone] + NAD+ = 2''-O-(2E)-but-2-enoyl-ADP-D-ribose + L-lysyl-[histone] + nicotinamide. Relationships: is a type of histone decrotonylase activity [GO:0160009]; is a type of NAD-dependent protein decrotonylase activity [GO:0160011] Also known as: NAD-dependent histone decrotonylase activity